mitochondrial tRNA 3'-end processing [GO:1990180] (biological process) Definition: The process in which the 3' end of a pre-tRNA molecule is converted to that of a mature tRNA in the mitochondrion. References: PMID:23928301 Sources: GOC:TermGenie, GOC:mah Also known as: tRNA 3' processing in mitochondria, tRNA 3' processing in mitochondrion, tRNA 3'-end processing in mitochondria Relationships: is a type of mitochondrial RNA 3'-end processing [GO:0000965]; is a type of GO:0042780; is a type of mitochondrial tRNA processing [GO:0090646]